{
  "gene": "UniProtKB:Q9NX52",
  "gene_symbol": "RHBDL2",
  "term_id": "GO:0004252",
  "gene_name": "Rhomboid-related protein 2",
  "term_label": "serine-type endopeptidase activity"
}